negative regulation of macrophage migration [GO:1905522] (biological process) Definition: Any process that stops, prevents or reduces the frequency, rate or extent of macrophage migration. References: PMID:25749876 Sources: GOC:TermGenie, GO_REF:0000058 Also known as: down regulation of macrophage migration, down-regulation of macrophage migration, downregulation of macrophage migration, inhibition of macrophage migration Relationships: is a type of negative regulation of mononuclear cell migration [GO:0071676]; is a type of regulation of macrophage migration [GO:1905521]; negatively regulates GO:1905517 Subtypes: negative regulation of macrophage chemotaxis [GO:0010760], negative regulation of microglial cell migration [GO:1904140]